T cell migration [GO:0072678] (biological process) Regulation: regulated by GO:2000404; negatively regulated by negative regulation of T cell migration [GO:2000405]; positively regulated by positive regulation of T cell migration [GO:2000406] Sources: CL:0000084, GOC:BHF, GOC:mah Relationships: is a type of lymphocyte migration [GO:0072676] Subtypes: T cell chemotaxis [GO:0010818], helper T cell diapedesis [GO:0035685], GO:0072679, GO:0072683, T cell meandering migration [GO:0120117] Also known as: T lymphocyte migration, T-cell migration, T-lymphocyte migration Definition: The movement of a T cell within or between different tissues and organs of the body.